{
  "term_id": "GO:0043408",
  "gene": "UniProtKB:Q13239",
  "term_label": "regulation of MAPK cascade",
  "gene_name": "Src-like-adapter",
  "gene_symbol": "SLA"
}